glycosylphosphatidylinositol-N-acetylglucosaminyltransferase (GPI-GnT) complex [GO:0000506] (cellular component) Definition: An enzyme complex that catalyzes the transfer of GlcNAc from UDP-GlcNAc to an acceptor phosphatidylinositol, the first step in the production of GPI anchors for cell surface proteins. The complex contains PIG-A, PIG-C, PIG-H, PIG-Q, PIG-P, and DPM2 in human, and Eri1p, Gpi1p, Gpi2p, Gpi15p, Gpi19p, and Spt14p in budding yeast. References: PMID:10944123, PMID:15163411 Sources: GOC:kp, GOC:rb Also known as: GPI-GlcNAc transferase complex, GPI-GnT complex, GPI-N-acetylglucosaminyltransferase complex Note: Note that this term should not be confused with 'GPI-anchor transamidase complex ; GO:0042765', which represents a distinct complex with a different catalytic activity. Relationships: is a type of membrane protein complex [GO:0098796]; is a type of endoplasmic reticulum protein-containing complex [GO:0140534]; is a type of GO:1990234; is part of endoplasmic reticulum membrane [GO:0005789]